{
  "term_label": "negative regulation of inflammatory response",
  "term_id": "GO:0050728",
  "gene_symbol": "PTGER4",
  "gene_name": "Prostaglandin E2 receptor EP4 subtype",
  "gene": "UniProtKB:P35408"
}